RNA 5'-gamma-phosphate methyltransferase activity [GO:1990276] (molecular function) References: PMID:22740346 Sources: GOC:al, GOC:vw Definition: Catalysis of the transfer of a methyl group from S-adenosyl-L-methionine to the 5'-gamma-phosphate in an RNA molecule. Also known as: RNA 5'-methyltransferase activity Relationships: is a type of GO:0008171; is a type of GO:0008173; is a type of S-adenosylmethionine-dependent methyltransferase activity [GO:0008757]